NADPH pyrophosphatase activity [GO:0010943] (MF) Definition: Catalysis of the reaction: NADPH + H2O = NMNH + ADP. Relationships: is a type of dinucleotide phosphatase activity [GO:0004551] References: PMID:12790796 Sources: GOC:tb, RHEA:60820